{
  "gene_symbol": "OTOP3",
  "gene": "UniProtKB:Q7RTS5",
  "gene_name": "Proton channel OTOP3",
  "term_id": "GO:0005886",
  "term_label": "plasma membrane"
}